agmatine kinase activity [GO:0047633] (molecular function) Sources: EC:2.7.3.10, RHEA:15953 Relationships: is_a kinase activity [GO:0016301]; is_a phosphotransferase activity, nitrogenous group as acceptor [GO:0016775] Definition: Catalysis of the reaction: agmatine + ATP = N(4)-phosphoagmatine + ADP + 3 H+. Also known as: ATP:agmatine 4-N-phosphotransferase activity, ATP:agmatine N4-phosphotransferase activity, phosphagen phosphokinase activity